blue light signaling pathway [GO:0009785] (BP) Definition: The series of molecular signals initiated upon sensing of blue light by photoreceptor molecule, at a wavelength between 400nm and 470nm. Sources: GOC:lr, GOC:sm Also known as: blue light signalling pathway Relationships: is a type of intracellular receptor signaling pathway [GO:0030522]; is a type of cellular response to blue light [GO:0071483]